{
  "term_id": "GO:0005669",
  "gene_name": "Transcription initiation factor TFIID subunit 4",
  "gene": "UniProtKB:O00268",
  "gene_symbol": "TAF4",
  "term_label": "transcription factor TFIID complex"
}